{
  "term_id": "GO:0009653",
  "gene_symbol": "FOXD2",
  "gene": "UniProtKB:O60548",
  "gene_name": "Forkhead box protein D2",
  "term_label": "anatomical structure morphogenesis"
}